{
  "gene_name": "Integrin alpha-6",
  "gene": "UniProtKB:P23229",
  "gene_symbol": "ITGA6",
  "term_id": "GO:0007229",
  "term_label": "integrin-mediated signaling pathway"
}